{
  "term_id": "GO:0071013",
  "term_label": "catalytic step 2 spliceosome",
  "gene_symbol": "SNRPB",
  "gene_name": "Small nuclear ribonucleoprotein-associated proteins B and B'",
  "gene": "UniProtKB:P14678"
}